{
  "gene": "UniProtKB:Q49A92",
  "term_id": "UNKNOWN:0003",
  "term_label": "Unknown cellular component",
  "gene_symbol": "C8orf34",
  "gene_name": "Uncharacterized protein C8orf34"
}